{
  "term_id": "GO:0005637",
  "gene": "UniProtKB:Q9UN42",
  "term_label": "nuclear inner membrane",
  "gene_symbol": "ATP1B4",
  "gene_name": "Protein ATP1B4"
}